{
  "gene": "UniProtKB:Q01804",
  "gene_symbol": "OTUD4",
  "gene_name": "OTU domain-containing protein 4",
  "term_id": "GO:0004843",
  "term_label": "cysteine-type deubiquitinase activity"
}